{
  "term_id": "UNKNOWN:0003",
  "gene": "UniProtKB:Q3MIW9",
  "gene_name": "Mucin-like protein 3",
  "term_label": "Unknown cellular component",
  "gene_symbol": "MUCL3"
}